coenzyme A metabolic process [GO:0015936] (biological process) Relationships: is a type of GO:0006753; is a type of sulfur compound metabolic process [GO:0006790]; is a type of amide metabolic process [GO:0043603]; is a type of GO:0072521 Also known as: CoA metabolism, coenzyme A metabolism Sources: ISBN:0198547684 Definition: The chemical reactions and pathways involving coenzyme A, 3'-phosphoadenosine-(5')diphospho(4')pantatheine, an acyl carrier in many acylation and acyl-transfer reactions in which the intermediate is a thiol ester. Subtypes: GO:0015937, GO:0015938